{
  "gene_symbol": "DNAJC19",
  "gene_name": "Mitochondrial import inner membrane translocase subunit TIM14",
  "term_label": "PAM complex, Tim23 associated import motor",
  "gene": "UniProtKB:Q96DA6",
  "term_id": "GO:0001405"
}